positive regulation of heterochromatin organization [GO:0120263] (biological process) Also known as: up regulation of heterochromatin organization, up-regulation of heterochromatin organization, upregulation of heterochromatin organization, activation of heterochromatin organization, stimulation of heterochromatin organization Relationships: is a type of regulation of heterochromatin organization [GO:0120261]; is a type of GO:1905269; positively regulates heterochromatin organization [GO:0070828] Definition: Any process that activates or increases the frequency, rate or extent of heterochromatin organization. Sources: GOC:krc